inositol phosphoceramide synthase activity [GO:0045140] (molecular function) Relationships: is a type of GO:0016758 References: PMID:9405490, PMID:9614099 Also known as: IPC synthase activity Regulation: RO_0002211 by GO:0070917 Definition: Catalysis of the reaction: phytoceramide + inositol phosphate = inositol phosphoceramide + diacylglycerol.